{
  "gene_name": "Low-density lipoprotein receptor",
  "gene_symbol": "LDLR",
  "term_label": "receptor-mediated endocytosis involved in cholesterol transport",
  "gene": "UniProtKB:P01130",
  "term_id": "GO:0090118"
}